{
  "term_id": "GO:0005654",
  "gene_symbol": "PPHLN1",
  "gene_name": "Periphilin-1",
  "term_label": "nucleoplasm",
  "gene": "UniProtKB:Q8NEY8"
}